{
  "term_label": "Unknown molecular function",
  "gene_name": "Platelet glycoprotein V",
  "gene": "UniProtKB:P40197",
  "term_id": "UNKNOWN:0001",
  "gene_symbol": "GP5"
}